exo-alpha-sialidase activity [GO:0004308] (molecular function) Regulation: regulated by modulation by host of viral exo-alpha-sialidase activity [GO:0044866]; positively regulated by GO:1903017 Definition: Catalysis of the hydrolysis of alpha-(2->3)-, alpha-(2->6)-, alpha-(2->8)-glycosidic linkages of terminal sialic residues in oligosaccharides, glycoproteins, glycolipids, colominic acid and synthetic substrates. Sources: EC:3.2.1.18 Relationships: is a type of GO:0016997 Also known as: N-acylneuraminate glycohydrolase activity, acetylneuraminidase activity, acetylneuraminyl hydrolase activity, alpha-neuraminidase activity, neuraminidase activity, sialidase activity